3-hydroxypimeloyl-CoA dehydrogenase activity [GO:0018464] (molecular function) Definition: Catalysis of the reaction: 3-hydroxypimelyl-CoA + NAD+ = 3-oxopimelyl-CoA + H+ + NADH. Sources: EC:1.1.1.259, RHEA:11168 Also known as: 3-hydroxypimeloyl-CoA:NAD+ oxidoreductase activity Relationships: is a type of oxidoreductase activity, acting on the CH-OH group of donors, NAD or NADP as acceptor [GO:0016616]